{
  "gene": "UniProtKB:Q9UKG9",
  "gene_symbol": "CROT",
  "term_id": "GO:0005777",
  "gene_name": "Peroxisomal carnitine O-octanoyltransferase",
  "term_label": "peroxisome"
}